cellobiose metabolic process [GO:2000891] (BP) Also known as: cellobiose metabolism Sources: GOC:mengo_curators Definition: The chemical reactions and pathways involving a cellobiose. Subtypes: GO:2000892 Relationships: is a type of GO:0005984